{
  "gene_symbol": "UST",
  "gene": "UniProtKB:Q9Y2C2",
  "gene_name": "Uronyl 2-sulfotransferase",
  "term_label": "Unknown biological process",
  "term_id": "UNKNOWN:0002"
}